{
  "gene_symbol": "TGFBR3",
  "gene_name": "Transforming growth factor beta receptor type 3",
  "gene": "UniProtKB:Q03167",
  "term_label": "regulation of transforming growth factor beta receptor signaling pathway",
  "term_id": "GO:0017015"
}